response to lipoic acid [GO:1903442] (BP) Relationships: is a type of response to fatty acid [GO:0070542] Subtypes: GO:1903443 References: PMID:23232760 Sources: GOC:TermGenie, GOC:sl, GO_REF:0000071 Definition: Any process that results in a change in state or activity of a cell or an organism (in terms of movement, secretion, enzyme production, gene expression, etc.) as a result of a lipoic acid stimulus.